{
  "term_label": "Unknown cellular component",
  "gene": "UniProtKB:Q8NET4",
  "gene_name": "Retrotransposon Gag-like protein 9",
  "gene_symbol": "RTL9",
  "term_id": "UNKNOWN:0003"
}